{
  "term_label": "Unknown biological process",
  "term_id": "UNKNOWN:0002",
  "gene_symbol": "TAF15",
  "gene": "UniProtKB:Q92804",
  "gene_name": "TATA-binding protein-associated factor 2N"
}